{
  "gene": "UniProtKB:Q8NA96",
  "gene_name": "Putative uncharacterized protein FLJ35723",
  "term_id": "UNKNOWN:0002",
  "gene_symbol": "Q8NA96",
  "term_label": "Unknown biological process"
}